{
  "gene_symbol": "USP38",
  "term_label": "cysteine-type deubiquitinase activity",
  "gene": "UniProtKB:Q8NB14",
  "gene_name": "Ubiquitin carboxyl-terminal hydrolase 38",
  "term_id": "GO:0004843"
}